{
  "gene": "UniProtKB:P19634",
  "gene_symbol": "SLC9A1",
  "term_id": "GO:0015385",
  "term_label": "sodium:proton antiporter activity",
  "gene_name": "Sodium_hydrogen exchanger 1"
}